morphine 6-dehydrogenase activity [GO:0050109] (molecular function) Also known as: morphine:NAD(P)+ 6-oxidoreductase activity, naloxone reductase activity, reductase, naloxone Definition: Catalysis of the reaction: morphine + NAD(P)+ = morphinone + NAD(P)H + H+. Relationships: is a type of oxidoreductase activity, acting on the CH-OH group of donors, NAD or NADP as acceptor [GO:0016616] Sources: EC:1.1.1.218, MetaCyc:MORPHINE-6-DEHYDROGENASE-RXN